{
  "term_id": "GO:0007059",
  "gene": "UniProtKB:Q6P1K2",
  "gene_name": "Polyamine-modulated factor 1",
  "gene_symbol": "PMF1",
  "term_label": "chromosome segregation"
}